{
  "gene_symbol": "BMP2KL",
  "term_id": "UNKNOWN:0002",
  "gene_name": "Putative BMP-2-inducible kinase-like protein",
  "term_label": "Unknown biological process",
  "gene": "UniProtKB:Q5H9B9"
}